endoplasmic reticulum-Golgi intermediate compartment (ERGIC) derived vesicle fusion with Golgi cis cisterna membrane [GO:1990689] (biological process) Definition: The joining of the lipid bilayer membrane around an ERGIC-derived vesicle to the lipid bilayer membrane around the Golgi cis cisterna. Such vesicles include COPII-coated transport vesicles involved in anterograde transport. Relationships: is a type of GO:0048280; is_a vesicle fusion with Golgi cis cisterna membrane [GO:1990670]; is part of endoplasmic reticulum to Golgi vesicle-mediated transport [GO:0006888] Also known as: ER-Golgi intermediate compartment derived vesicle fusion with Golgi cis cisterna membrane, ER-Golgi intermediate compartment derived vesicle fusion with cis-Golgi cisterna membrane, ERGIC-derived vesicle fusion with Golgi cis cisterna membrane, ERGIC-derived vesicle fusion with cis-Golgi cisterna membrane, endoplasmic reticulum-Golgi intermediate compartment (ERGIC) derived vesicle fusion with cis-Golgi cisterna membrane References: PMID:16038056, PMID:24119662 Sources: GOC:bhm